{
  "term_id": "GO:0005634",
  "term_label": "nucleus",
  "gene_name": "Cyclic AMP-responsive element-binding protein 3",
  "gene_symbol": "CREB3",
  "gene": "UniProtKB:O43889"
}